glycerol to glycerone phosphate metabolic process [GO:0061610] (biological process) Also known as: glycerol metabolism to DHAP, glycerol metabolism to dihydroxyacetone phosphate, glycerol metabolism to glycerone phosphate, glycerol to DHAP metabolic process, glycerol to dihydroxyacetone phosphate metabolic process Sources: GOC:dph, ISBN:0201090910 Definition: The chemical reactions and pathways in which glycerol, 1,2,3-propanetriol, is converted to glycerone phosphate. Relationships: is a type of glycerol metabolic process [GO:0006071]; is a type of phosphate-containing compound metabolic process [GO:0006796]; is a type of organophosphate metabolic process [GO:0019637]; is a type of primary alcohol metabolic process [GO:0034308]; is a type of ketone metabolic process [GO:0042180]; is a type of carbohydrate derivative metabolic process [GO:1901135]; BFO_0000051 glycerol kinase activity [GO:0004370]; has part GO:0141152